high-affinity basic amino acid transmembrane transporter activity [GO:0005287] (molecular function) Sources: GOC:mtg_transport Subtypes: high-affinity L-arginine transmembrane transporter activity [GO:0005289], high-affinity L-histidine transmembrane transporter activity [GO:0005291], high-affinity lysine transmembrane transporter activity [GO:0005292], GO:0015330 Relationships: is a type of basic amino acid transmembrane transporter activity [GO:0015174] Also known as: high-affinity basic amino acid transporter activity, high affinity basic amino acid transmembrane transporter activity Definition: Enables the transfer of basic amino acids from one side of a membrane to the other. Acidic amino acids have a pH above 7. In high-affinity transport the transporter is able to bind the solute even if it is only present at very low concentrations.